epinephrine secretion [GO:0048242] (biological process) Subtypes: epinephrine secretion, neurotransmission [GO:0061529] Definition: The regulated release of epinephrine by a cell. Epinephrine is a catecholamine hormone secreted by the adrenal medulla and a neurotransmitter, released by certain neurons and active in the central nervous system. Sources: GOC:ef, GOC:jid Regulation: regulated by regulation of epinephrine secretion [GO:0014060]; negatively regulated by GO:0032811; RO_0002213 by positive regulation of epinephrine secretion [GO:0032812] Also known as: adrenaline secretion Relationships: is_a epinephrine transport [GO:0048241]; is a type of catecholamine secretion [GO:0050432]